CCG codon-amino acid adaptor activity [GO:0033424] (molecular function) Note: Note that in the standard genetic code, CCG codes for proline. Also known as: proline tRNA Definition: A triplet codon-amino acid adaptor activity that recognizes a CCG codon. Relationships: is a type of triplet codon-amino acid adaptor activity [GO:0030533] Sources: GOC:mah